{
  "gene_symbol": "RHOD",
  "gene_name": "Rho-related GTP-binding protein RhoD",
  "gene": "UniProtKB:O00212",
  "term_id": "UNKNOWN:0003",
  "term_label": "Unknown cellular component"
}